Golgi membrane coat protein complex assembly [GO:0048197] (biological process) Definition: The aggregation, arrangement and bonding together of priming complexes to form a coat on a Golgi membrane. Priming complexes associate laterally and additional coat proteins are recruited from the cytosol to the forming coat. Cargo proteins diffuse into the budding site and become trapped by their interactions with the coat. Also known as: Golgi apparatus membrane coat protein complex assembly, Golgi membrane bud coat oligomerisation, dictyosome membrane binding by cytosolic coat proteins, dictyosome membrane bud coat oligomerisation References: PMID:10219233 Sources: GOC:jid, GOC:mah, ISBN:0716731363 Relationships: is a type of protein-containing complex assembly [GO:0065003]; is part of Golgi transport vesicle coating [GO:0048200]